{
  "gene": "UniProtKB:Q6UXZ0",
  "gene_symbol": "TMIGD1",
  "gene_name": "Transmembrane and immunoglobulin domain-containing protein 1",
  "term_id": "GO:0043005",
  "term_label": "neuron projection"
}